L-phenylalanine transmembrane transporter activity [GO:0015192] (molecular function) Relationships: is a type of aromatic amino acid transmembrane transporter activity [GO:0015173]; is a type of L-amino acid transmembrane transporter activity [GO:0015179]; is part of phenylalanine transport [GO:0015823] Sources: GOC:ai, GOC:mtg_transport, ISBN:0815340729 Also known as: L-phenylalanine transporter activity, L-phenylalanine permease activity Definition: Enables the transfer of L-phenylalanine from one side of a membrane to the other. L-phenylalanine is 2-amino-3-phenylpropanoic acid.